{
  "term_id": "UNKNOWN:0001",
  "gene_symbol": "COX5A",
  "gene_name": "Cytochrome c oxidase subunit 5A, mitochondrial",
  "term_label": "Unknown molecular function",
  "gene": "UniProtKB:P20674"
}